establishment of anatomical structure orientation [GO:0048560] (biological process) Relationships: is a type of axis specification [GO:0009798]; is part of anatomical structure morphogenesis [GO:0009653] Subtypes: establishment of animal organ orientation [GO:0048561], establishment of plant organ orientation [GO:0090707] Definition: The process that determines the orientation of an anatomical structure with reference to an axis. Sources: GOC:jid